chemotaxis to cAMP [GO:0043327] (biological process) Definition: The directed movement of a motile cell or organism in response to the presence of 3',5'-cAMP. Also known as: chemotaxis to 3',5' cAMP, chemotaxis to 3',5'-cAMP, chemotaxis to adenosine 3',5'-cyclophosphate, chemotaxis to cyclic AMP Relationships: is a type of chemotaxis [GO:0006935] Sources: GOC:go_curators Regulation: regulated by regulation of positive chemotaxis to cAMP [GO:0061118]; positively regulated by positive regulation of positive chemotaxis to cAMP [GO:0061122]; negatively regulated by negative regulation of positive chemotaxis to cAMP [GO:0061123]